male pronuclear envelope synthesis [GO:0035043] (biological process) Definition: Assembly of a nuclear envelope containing nuclear pores and a lamina around the male pronucleus, the final step in sperm pronuclear formation. Relationships: is a type of pronuclear envelope synthesis [GO:0018985]; is part of male pronucleus assembly [GO:0035039] References: PMID:11735001 Sources: GOC:bf